{
  "gene_symbol": "ETDB",
  "gene_name": "Embryonic testis differentiation protein homolog B",
  "term_id": "UNKNOWN:0002",
  "term_label": "Unknown biological process",
  "gene": "UniProtKB:P0DPP9"
}